{
  "gene_symbol": "ZNRF1",
  "gene_name": "E3 ubiquitin-protein ligase ZNRF1",
  "term_label": "protein K48-linked ubiquitination",
  "gene": "UniProtKB:Q8ND25",
  "term_id": "GO:0070936"
}